{
  "term_label": "cohesin unloader activity",
  "gene_name": "Sister chromatid cohesion protein PDS5 homolog B",
  "gene_symbol": "PDS5B",
  "term_id": "GO:0140670",
  "gene": "UniProtKB:Q9NTI5"
}